{
  "gene": "UniProtKB:Q8WWF5",
  "gene_symbol": "ZNRF4",
  "term_label": "ubiquitin-dependent protein catabolic process",
  "term_id": "GO:0006511",
  "gene_name": "E3 ubiquitin-protein ligase ZNRF4"
}